negative regulation of spermidine biosynthetic process [GO:1901305] (biological process) Relationships: is a type of negative regulation of polyamine biosynthetic process [GO:0170066]; is a type of regulation of spermidine biosynthetic process [GO:1901304]; negatively regulates spermidine biosynthetic process [GO:0008295] Also known as: down regulation of spermidine anabolism, down regulation of spermidine biosynthesis, down regulation of spermidine biosynthetic process, down regulation of spermidine formation, down regulation of spermidine synthesis, down-regulation of spermidine anabolism, down-regulation of spermidine biosynthesis, down-regulation of spermidine biosynthetic process, down-regulation of spermidine formation, down-regulation of spermidine synthesis, downregulation of spermidine anabolism, downregulation of spermidine biosynthesis, downregulation of spermidine biosynthetic process, downregulation of spermidine formation, downregulation of spermidine synthesis, inhibition of spermidine anabolism, inhibition of spermidine biosynthesis, inhibition of spermidine formation, inhibition of spermidine synthesis, negative regulation of spermidine anabolism, negative regulation of spermidine biosynthesis, negative regulation of spermidine formation, negative regulation of spermidine synthesis, inhibition of spermidine biosynthetic process Definition: Any process that stops, prevents or reduces the frequency, rate or extent of spermidine biosynthetic process. Sources: GOC:TermGenie, GOC:pm